exonucleolytic trimming to generate mature 3'-end of 5.8S rRNA from tricistronic rRNA transcript (SSU-rRNA, 5.8S rRNA, LSU-rRNA) [GO:0000467] (biological process) References: PMID:10690410 Sources: GOC:krc Relationships: is a type of rRNA 3'-end processing [GO:0031125]; is part of maturation of 5.8S rRNA from tricistronic rRNA transcript (SSU-rRNA, 5.8S rRNA, LSU-rRNA) [GO:0000466] Definition: Exonucleolytic digestion of a pre-rRNA molecule to generate the mature 3'-end of a 5.8S rRNA molecule derived from an originally tricistronic pre-rRNA transcript that contained the Small Subunit (SSU) rRNA, the 5.8S rRNA, and the Large Subunit (LSU) rRNA in that order from 5' to 3' along the primary transcript.